{
  "term_label": "signaling receptor activity",
  "gene_name": "Killer cell lectin-like receptor subfamily B member 1",
  "gene": "UniProtKB:Q12918",
  "gene_symbol": "KLRB1",
  "term_id": "GO:0038023"
}